{
  "term_id": "GO:0016139",
  "gene_name": "Alpha-N-acetylgalactosaminidase",
  "term_label": "glycoside catabolic process",
  "gene": "UniProtKB:P17050",
  "gene_symbol": "NAGA"
}